{
  "gene_symbol": "SNTB2",
  "term_id": "UNKNOWN:0001",
  "gene": "UniProtKB:Q13425",
  "term_label": "Unknown molecular function",
  "gene_name": "Beta-2-syntrophin"
}